medium-chain fatty acyl-CoA oxidase activity [GO:0120523] (molecular function) Note: While there is not universal consensus on the lengths of short-, medium-, long- and very-long-chain fatty acids, the GO uses the definitions in ChEBI (see CHEBI:26666, CHEBI:59554, CHEBI:15904 and CHEBI:27283). Relationships: is a type of acyl-CoA oxidase activity [GO:0003997] Definition: Catalysis of the reaction: a medium-chain 2,3-saturated fatty acyl-CoA + O2 = a medium-chain (2E)-enoyl-CoA + H2O2. Sources: RHEA:78855